MutS complex [GO:1990710] (cellular component) Also known as: MutS mismatch repair complex References: PMID:21666597 Sources: GOC:bhm Relationships: is a type of mismatch repair complex [GO:0032300]; is a type of DNA repair complex [GO:1990391] Definition: A homodimeric mismatch repair complex involved in binding to and correcting insertion/deletion mutations. Note: An example of this is MutS in E. coli (UniProt symbol P23909) in PMID:21666597 (inferred from physical interaction).